threonine metabolic process [GO:0006566] (biological process) Definition: The chemical reactions and pathways involving threonine (2-amino-3-hydroxybutyric acid), a polar, uncharged, essential amino acid found in peptide linkage in proteins. Also known as: methionine and threonine metabolic process, methionine and threonine metabolism, threonine metabolism Relationships: is a type of carboxylic acid metabolic process [GO:0019752] Sources: GOC:jl, ISBN:0198506732 Subtypes: GO:0006567, threonine biosynthetic process [GO:0009088]